{
  "gene_name": "Beta-catenin-interacting protein 1",
  "gene_symbol": "CTNNBIP1",
  "term_label": "cytosol",
  "gene": "UniProtKB:Q9NSA3",
  "term_id": "GO:0005829"
}